{
  "gene_symbol": "LASP1NB",
  "term_id": "UNKNOWN:0002",
  "gene": "UniProtKB:A0A1B0GWH6",
  "term_label": "Unknown biological process",
  "gene_name": "LASP1 neighbor protein"
}